zeta DNA polymerase complex [GO:0016035] (cellular component) References: PMID:16631579, PMID:16971464 Definition: A heterodimeric DNA polymerase complex that catalyzes error-prone DNA synthesis in contexts such as translesion synthesis and double-stranded break repair. First characterized in Saccharomyces, in which the subunits are Rev3p and Rev7p; a third protein, Rev1p, is often associated with the polymerase dimer. Relationships: is a type of GO:0042575